{
  "term_label": "SCF ubiquitin ligase complex",
  "gene_symbol": "FBXL14",
  "term_id": "GO:0019005",
  "gene": "UniProtKB:Q8N1E6",
  "gene_name": "F-box_LRR-repeat protein 14"
}